{
  "gene_symbol": "LDHB",
  "gene": "UniProtKB:P07195",
  "term_label": "lactate metabolic process",
  "gene_name": "L-lactate dehydrogenase B chain",
  "term_id": "GO:0006089"
}